{
  "term_label": "transcription factor TFIID complex",
  "gene_name": "Transcription initiation factor TFIID subunit 7",
  "term_id": "GO:0005669",
  "gene": "UniProtKB:Q15545",
  "gene_symbol": "TAF7"
}